3',4',5'-trimethylmyricetin 7-O-methyltransferase activity [GO:0102439] (molecular function) Definition: Catalysis of the reaction: 3',4',5'-O-trimethylmyricetin + S-adenosyl-L-methionine = 7,3',4',5'-O-tetramethylmyricetin + S-adenosyl-L-homocysteine. Sources: RHEA:74739 Relationships: is a type of methyltransferase activity [GO:0008168]